{
  "term_label": "DNA-binding transcription factor activity",
  "term_id": "GO:0003700",
  "gene": "UniProtKB:Q9NQV5",
  "gene_name": "PR domain-containing protein 11",
  "gene_symbol": "PRDM11"
}